7,8-dihydro-D-neopterin 2',3'-cyclic phosphate phosphodiesterase activity [GO:0044688] (molecular function) Definition: Catalysis of the reaction: 7,8-dihydro-D-neopterin 2',3'-cyclic phosphate + H2O = 7,8-dihydroneopterin 3'-phosphate + H+. References: PMID:19746965 Sources: GOC:mengo_curators Relationships: is a type of phosphoric diester hydrolase activity [GO:0008081]; is part of GO:2001116